{
  "gene_name": "3-keto-steroid reductase_17-beta-hydroxysteroid dehydrogenase 7",
  "gene": "UniProtKB:P56937",
  "term_label": "estradiol 17-beta-dehydrogenase [NAD(P)+] activity",
  "term_id": "GO:0004303",
  "gene_symbol": "HSD17B7"
}